{
  "gene_symbol": "PIWIL4",
  "term_id": "GO:0004521",
  "gene": "UniProtKB:Q7Z3Z4",
  "term_label": "RNA endonuclease activity",
  "gene_name": "Piwi-like protein 4"
}